{
  "term_id": "UNKNOWN:0002",
  "term_label": "Unknown biological process",
  "gene": "UniProtKB:Q9BYZ8",
  "gene_name": "Regenerating islet-derived protein 4",
  "gene_symbol": "REG4"
}